{
  "gene_name": "WAP four-disulfide core domain protein 1",
  "term_label": "Unknown molecular function",
  "term_id": "UNKNOWN:0001",
  "gene_symbol": "WFDC1",
  "gene": "UniProtKB:Q9HC57"
}